{
  "gene": "UniProtKB:O43166",
  "gene_name": "Signal-induced proliferation-associated 1-like protein 1",
  "gene_symbol": "SIPA1L1",
  "term_label": "actin cytoskeleton organization",
  "term_id": "GO:0030036"
}